negative regulation of maintenance of meiotic sister chromatid cohesion [GO:0034095] (biological process) Sources: GOC:mah, GOC:vw Subtypes: negative regulation of maintenance of meiotic sister chromatid cohesion, centromeric [GO:2000710] Relationships: is a type of negative regulation of maintenance of sister chromatid cohesion [GO:0034092]; is a type of regulation of maintenance of meiotic sister chromatid cohesion [GO:0034094]; negatively regulates GO:0034090 Definition: Any process that decreases the extent to which the association between sister chromatids of a replicated chromosome is maintained during a meiotic cell cycle.